{
  "gene_symbol": "ATP8B1",
  "gene_name": "Phospholipid-transporting ATPase IC",
  "gene": "UniProtKB:O43520",
  "term_label": "Golgi organization",
  "term_id": "GO:0007030"
}